{
  "gene": "UniProtKB:Q9GZU5",
  "gene_symbol": "NYX",
  "term_label": "extracellular matrix",
  "gene_name": "Nyctalopin",
  "term_id": "GO:0031012"
}